{
  "term_label": "Cul2-RING ubiquitin ligase complex",
  "term_id": "GO:0031462",
  "gene_name": "Putative PRAME family member 13",
  "gene_symbol": "PRAMEF13",
  "gene": "UniProtKB:Q5VWM6"
}